{
  "term_label": "nucleus",
  "gene_symbol": "USP7",
  "gene_name": "Ubiquitin carboxyl-terminal hydrolase 7",
  "gene": "UniProtKB:Q93009",
  "term_id": "GO:0005634"
}